{
  "gene": "UniProtKB:P50148",
  "term_id": "GO:0031683",
  "term_label": "G-protein beta/gamma-subunit complex binding",
  "gene_name": "Guanine nucleotide-binding protein G(q) subunit alpha",
  "gene_symbol": "GNAQ"
}